regulation of naphtho-gamma-pyrone biosynthetic process [GO:1900846] (biological process) Definition: Any process that modulates the frequency, rate or extent of naphtho-gamma-pyrone biosynthetic process. Subtypes: negative regulation of naphtho-gamma-pyrone biosynthetic process [GO:1900847], positive regulation of naphtho-gamma-pyrone biosynthetic process [GO:1900848] Sources: GOC:TermGenie, GOC:di Relationships: is a type of GO:0010566; regulates GO:1900787 Also known as: regulation of naphtho-gamma-pyrone anabolism, regulation of naphtho-gamma-pyrone biosynthesis, regulation of naphtho-gamma-pyrone formation, regulation of naphtho-gamma-pyrone synthesis, regulation of naphtho-gamma-pyrones anabolism, regulation of naphtho-gamma-pyrones biosynthesis, regulation of naphtho-gamma-pyrones biosynthetic process, regulation of naphtho-gamma-pyrones formation, regulation of naphtho-gamma-pyrones synthesis